{
  "gene": "UniProtKB:Q8N3D4",
  "term_label": "actin filament binding",
  "gene_symbol": "EHBP1L1",
  "term_id": "GO:0051015",
  "gene_name": "EH domain-binding protein 1-like protein 1"
}